positive regulation of (1->3)-beta-D-glucan biosynthetic process [GO:0060635] (biological process) Sources: GOC:dph, GOC:tb Relationships: is a type of positive regulation of macromolecule biosynthetic process [GO:0010557]; is a type of GO:0032953; is a type of GO:0045913; positively regulates GO:0006075 Subtypes: positive regulation of regulation of ascospore wall (1->3)-beta-D-glucan biosynthetic process [GO:0140748] Also known as: positive regulation of 1,3-beta-D-glucan biosynthetic process Definition: Any process that increases the frequency, rate or extent of the chemical reactions and pathways resulting in the formation of (1->3)-beta-D-glucans.